regulation of cell adhesion involved in intussusceptive angiogenesis [GO:0002045] (BP) Definition: The process that modulates the frequency, rate or extent of attachment of a blood vessel endothelial cell to another cell or to the extracellular matrix involved in intussusceptive angiogenesis. Relationships: is a type of regulation of cell adhesion [GO:0030155]; is part of GO:0002041 References: PMID:16391003